{
  "term_label": "nucleus",
  "gene": "UniProtKB:Q92870",
  "term_id": "GO:0005634",
  "gene_symbol": "APBB2",
  "gene_name": "Amyloid beta precursor protein binding family B member 2"
}